carbon catabolite repression of transcription from RNA polymerase II promoter [GO:0000437] (biological process) Relationships: is a type of negative regulation of transcription by RNA polymerase II [GO:0000122]; is a type of GO:0000429; is a type of carbon catabolite repression of transcription [GO:0045013] Sources: GOC:krc Definition: A transcription regulation process in which the presence of one carbon source leads to a decrease in the frequency, rate, or extent of transcription, from an RNA polymerase II promoter, of specific genes involved in the metabolism of other carbon sources. Subtypes: GO:0000434, negative regulation of transcription from RNA polymerase II promoter by a nonfermentable carbon source [GO:0061415] Also known as: negative regulation of transcription from RNA polymerase II promoter by carbon catabolites